maintenance of sister chromatid cohesion [GO:0034086] (BP) Definition: The process in which the association between sister chromatids of a replicated chromosome is maintained as chromosomes condense, attach to the spindle in a bipolar orientation, and congress to the metaphase plate. References: PMID:14623866 Sources: GOC:mah Relationships: is a type of GO:0022402; is part of sister chromatid cohesion [GO:0007062] Subtypes: maintenance of mitotic sister chromatid cohesion [GO:0034088], GO:0034090 Regulation: regulated by regulation of maintenance of sister chromatid cohesion [GO:0034091]; negatively regulated by negative regulation of maintenance of sister chromatid cohesion [GO:0034092]; positively regulated by positive regulation of maintenance of sister chromatid cohesion [GO:0034093]